positive regulation of bone development [GO:1903012] (biological process) References: PMID:22510437 Sources: GOC:TermGenie, GOC:mr, GO_REF:0000058 Definition: Any process that activates or increases the frequency, rate or extent of bone development. Relationships: is_a positive regulation of developmental process [GO:0051094]; is a type of positive regulation of multicellular organismal process [GO:0051240]; is a type of GO:1903010; positively regulates bone development [GO:0060348] Also known as: up regulation of bone development, up-regulation of bone development, upregulation of bone development, activation of bone development